{
  "gene_symbol": "L1CAM",
  "term_label": "synapse organization",
  "gene_name": "Neural cell adhesion molecule L1",
  "term_id": "GO:0050808",
  "gene": "UniProtKB:P32004"
}